descending aorta morphogenesis [GO:0035911] (biological process) Relationships: is_a anatomical structure morphogenesis [GO:0009653]; is part of GO:0035906; is part of GO:0035909 Definition: The process in which the anatomical structures of the descending aorta are generated and organized. The descending aorta is the portion of the aorta in a two-pass circulatory system from the arch of aorta to the point where it divides into the common iliac arteries. In a two-pass circulatory system blood passes twice through the heart to supply the body once. Sources: GOC:bf, GOC:dgh, MA:0002571, UBERON:0001514, Wikipedia:Descending_aorta